{
  "gene_symbol": "PRIMPOL",
  "term_id": "GO:0003887",
  "term_label": "DNA-directed DNA polymerase activity",
  "gene": "UniProtKB:Q96LW4",
  "gene_name": "DNA-directed primase_polymerase protein"
}